{
  "term_label": "signal transduction",
  "gene": "UniProtKB:Q9Y572",
  "gene_name": "Receptor-interacting serine_threonine-protein kinase 3",
  "term_id": "GO:0007165",
  "gene_symbol": "RIPK3"
}